{
  "term_label": "sperm principal piece",
  "term_id": "GO:0097228",
  "gene_symbol": "CATSPER4",
  "gene": "UniProtKB:Q7RTX7",
  "gene_name": "Cation channel sperm-associated protein 4"
}